animal organ development [GO:0048513] (biological process) Relationships: is a type of GO:0048856 Definition: Development of a tissue or tissues that work together to perform a specific function or functions. Development pertains to the process whose specific outcome is the progression of a structure over time, from its formation to the mature structure. Organs are commonly observed as visibly distinct structures, but may also exist as loosely associated clusters of cells that work together to perform a specific function or functions. Also known as: development of an organ, organogenesis Subtypes: GO:0001822, GO:0001890, ventral cord development [GO:0007419], brain development [GO:0007420], sensory organ development [GO:0007423], imaginal disc development [GO:0007444], fat body development [GO:0007503], heart development [GO:0007507], muscle organ development [GO:0007517], gonad development [GO:0008406], respiratory tube development [GO:0030323], lung development [GO:0030324], pancreas development [GO:0031016], animal organ regeneration [GO:0031100], vulval development [GO:0040025], skin development [GO:0043588], hematopoietic or lymphoid organ development [GO:0048534], embryonic organ development [GO:0048568], proboscis development [GO:0048728], gland development [GO:0048732], swim bladder development [GO:0048794], genitalia development [GO:0048806], cartilage development [GO:0051216], GO:0060065, GO:0060157, bone development [GO:0060348], GO:0060438, gallbladder development [GO:0061010], urethra development [GO:0061068], Malpighian tubule development [GO:0072002], ureter development [GO:0072189], larynx development [GO:0120224] Sources: GOC:dph, GOC:jid